polyamine transmembrane transport [GO:1902047] (biological process) Subtypes: spermine transmembrane transport [GO:1903710], spermidine transmembrane transport [GO:1903711] Definition: The process in which a polyamine macromolecule is transported across a membrane. Sources: GOC:TermGenie, GOC:vw Also known as: polyamine import, polyamine uptake Relationships: is a type of GO:0015846; is a type of transmembrane transport [GO:0055085] Regulation: regulated by regulation of polyamine transmembrane transport [GO:1902267]; negatively regulated by GO:1902268; positively regulated by positive regulation of polyamine transmembrane transport [GO:1902269]